{
  "gene_name": "Protocadherin-19",
  "gene_symbol": "PCDH19",
  "term_id": "GO:0050839",
  "gene": "UniProtKB:Q8TAB3",
  "term_label": "cell adhesion molecule binding"
}